negative regulation of convergent extension involved in axis elongation [GO:1901233] (biological process) Relationships: is a type of negative regulation of developmental growth [GO:0048640]; is a type of regulation of convergent extension involved in axis elongation [GO:1901232]; is a type of negative regulation of morphogenesis of an epithelium [GO:1905331]; negatively regulates GO:0060028 Subtypes: negative regulation of convergent extension involved in somitogenesis [GO:1904128] Definition: Any process that stops, prevents or reduces the frequency, rate or extent of convergent extension involved in axis elongation. Sources: GOC:BHF, GOC:TermGenie Also known as: down regulation of convergent extension involved in axis elongation, down-regulation of convergent extension involved in axis elongation, downregulation of convergent extension involved in axis elongation, inhibition of convergent extension involved in axis elongation